{
  "term_label": "RNA polymerase II, core complex",
  "gene_symbol": "TUFT1",
  "term_id": "GO:0005665",
  "gene": "UniProtKB:Q9NNX1",
  "gene_name": "Tuftelin"
}